{
  "gene_name": "Receptor-type tyrosine-protein kinase FLT3",
  "term_id": "GO:0016477",
  "term_label": "cell migration",
  "gene": "UniProtKB:P36888",
  "gene_symbol": "FLT3"
}